{
  "gene_symbol": "CTSK",
  "gene_name": "Cathepsin K",
  "gene": "UniProtKB:P43235",
  "term_id": "GO:0005764",
  "term_label": "lysosome"
}